{
  "term_label": "positive regulation of MAPK cascade",
  "gene_symbol": "ERBB4",
  "term_id": "GO:0043410",
  "gene": "UniProtKB:Q15303",
  "gene_name": "Receptor tyrosine-protein kinase erbB-4"
}